{
  "gene_symbol": "CEBPA",
  "term_label": "RNA polymerase II cis-regulatory region sequence-specific DNA binding",
  "gene": "UniProtKB:P49715",
  "gene_name": "CCAAT_enhancer-binding protein alpha",
  "term_id": "GO:0000978"
}